{
  "gene": "UniProtKB:Q8NGJ5",
  "gene_name": "Olfactory receptor 51L1",
  "gene_symbol": "OR51L1",
  "term_id": "GO:0004984",
  "term_label": "olfactory receptor activity"
}